{
  "term_id": "GO:0000981",
  "gene": "UniProtKB:P52738",
  "gene_symbol": "ZNF140",
  "term_label": "DNA-binding transcription factor activity, RNA polymerase II-specific",
  "gene_name": "Zinc finger protein 140"
}